{
  "term_id": "GO:0001501",
  "gene": "UniProtKB:P50281",
  "gene_symbol": "MMP14",
  "term_label": "skeletal system development",
  "gene_name": "Matrix metalloproteinase-14"
}